{
  "gene_name": "Adrenocortical dysplasia protein homolog",
  "term_label": "protein localization to chromosome, telomeric region",
  "gene": "UniProtKB:Q96AP0",
  "term_id": "GO:0070198",
  "gene_symbol": "ACD"
}